{
  "gene_name": "Alkaline ceramidase 1",
  "term_id": "GO:0046512",
  "gene": "UniProtKB:Q8TDN7",
  "term_label": "sphingosine biosynthetic process",
  "gene_symbol": "ACER1"
}